{
  "gene": "UniProtKB:Q86XQ3",
  "term_label": "CatSper complex",
  "term_id": "GO:0036128",
  "gene_name": "Cation channel sperm-associated protein 3",
  "gene_symbol": "CATSPER3"
}